{
  "gene_name": "Ankyrin repeat domain-containing protein 1",
  "term_label": "regulation of transcription by RNA polymerase II",
  "gene": "UniProtKB:Q15327",
  "gene_symbol": "ANKRD1",
  "term_id": "GO:0006357"
}